alpha1-beta1 integrin-alpha3(VI) complex [GO:0070465] (cellular component) References: PMID:8387021 Also known as: ITGA1-ITGB1-COL6A3 complex Relationships: is a type of plasma membrane protein complex [GO:0098797] Definition: A protein complex that consists of an alpha1-beta1 integrin complex bound to a type VI collagen triple helix containing an alpha3(VI) chain.